host cell plasmodesma [GO:0044219] (cellular component) Definition: A fine cytoplasmic channel, found in all higher plants, that connects the cytoplasm of one host cell to that of an adjacent host cell. Relationships: is a type of host cell junction [GO:0044156] References: PMID:16903353 Sources: GOC:rph